{
  "gene_symbol": "CPEB2",
  "term_id": "GO:0005634",
  "gene_name": "Cytoplasmic polyadenylation element-binding protein 2",
  "term_label": "nucleus",
  "gene": "UniProtKB:Q7Z5Q1"
}